kinase binding [GO:0019900] (molecular function) Definition: Binding to a kinase, any enzyme that catalyzes the transfer of a phosphate group. Sources: GOC:jl Relationships: is a type of enzyme binding [GO:0019899] Subtypes: protein kinase binding [GO:0019901], GO:0036313